{
  "gene": "UniProtKB:O00628",
  "term_label": "peroxisomal matrix",
  "gene_name": "Peroxisomal targeting signal 2 receptor",
  "term_id": "GO:0005782",
  "gene_symbol": "PEX7"
}